vulval cell fate determination [GO:0072326] (biological process) Relationships: is a type of cell fate determination [GO:0001709]; is part of GO:0072325 Definition: The process in which a cell becomes capable of differentiating autonomously into a nematode vulval cell regardless of its environment; upon determination, the cell fate cannot be reversed. In nematodes, the vulva is formed from ventral epidermal cells during larval stages to give rise to a fully formed adult vulva, which is the egg-laying organ of female and hermaphrodite nematodes. References: PMID:11236714 Sources: GOC:kmv, GOC:mah, ISBN:087969307X